{
  "gene_name": "Dynactin subunit 1",
  "term_label": "Unknown molecular function",
  "term_id": "UNKNOWN:0001",
  "gene": "UniProtKB:Q14203",
  "gene_symbol": "DCTN1"
}